{
  "gene": "UniProtKB:Q9NR90",
  "term_label": "3'-UTR-mediated mRNA stabilization",
  "gene_name": "Deleted in azoospermia protein 3",
  "term_id": "GO:0070935",
  "gene_symbol": "DAZ3"
}